{
  "gene_name": "Leucine-zipper-like transcriptional regulator 1",
  "term_label": "Cul3-RING ubiquitin ligase complex",
  "gene_symbol": "LZTR1",
  "gene": "UniProtKB:Q8N653",
  "term_id": "GO:0031463"
}